{
  "gene_symbol": "IRF4",
  "term_id": "GO:0006357",
  "term_label": "regulation of transcription by RNA polymerase II",
  "gene_name": "Interferon regulatory factor 4",
  "gene": "UniProtKB:Q15306"
}